{
  "gene_name": "Aldo-keto reductase family 1 member C1",
  "gene_symbol": "AKR1C1",
  "term_id": "GO:0032052",
  "term_label": "bile acid binding",
  "gene": "UniProtKB:Q04828"
}